{
  "term_label": "extracellular space",
  "term_id": "GO:0005615",
  "gene": "UniProtKB:Q14508",
  "gene_name": "WAP four-disulfide core domain protein 2",
  "gene_symbol": "WFDC2"
}